{
  "gene_symbol": "SIGLEC16",
  "term_id": "GO:0005886",
  "term_label": "plasma membrane",
  "gene_name": "Sialic acid-binding Ig-like lectin 16",
  "gene": "UniProtKB:A6NMB1"
}